{
  "gene_symbol": "FCN3",
  "gene": "UniProtKB:O75636",
  "term_label": "carbohydrate derivative binding",
  "gene_name": "Ficolin-3",
  "term_id": "GO:0097367"
}